{
  "term_label": "GTPase activator activity",
  "term_id": "GO:0005096",
  "gene_symbol": "TBC1D15",
  "gene_name": "TBC1 domain family member 15",
  "gene": "UniProtKB:Q8TC07"
}